acquisition of nutrients from host [GO:0044002] (biological process) Sources: GOC:cc, GOC:jl Definition: The process that begins with the production and formation of structures and molecules in an organism that are required for the acquisition and utilization of nutrients from its host organism, and the ends with the acquirement of the nutrients. The host is defined as the larger of the organisms involved in a symbiotic interaction. Relationships: is a type of biological process involved in interaction with host [GO:0051701] Subtypes: iron acquisition from host [GO:0044847], GO:0052091